{
  "term_id": "GO:0055085",
  "gene_name": "Probable UDP-sugar transporter protein SLC35A5",
  "term_label": "transmembrane transport",
  "gene": "UniProtKB:Q9BS91",
  "gene_symbol": "SLC35A5"
}